{
  "gene_name": "Protein GAPT",
  "gene": "UniProtKB:Q8N292",
  "gene_symbol": "GAPT",
  "term_id": "GO:0001782",
  "term_label": "B cell homeostasis"
}